{
  "term_id": "GO:0006511",
  "gene_name": "E3 ubiquitin-protein ligase parkin",
  "term_label": "ubiquitin-dependent protein catabolic process",
  "gene_symbol": "PRKN",
  "gene": "UniProtKB:O60260"
}